{
  "gene_symbol": "KIF15",
  "term_label": "microtubule motor activity",
  "gene_name": "Kinesin-like protein KIF15",
  "gene": "UniProtKB:Q9NS87",
  "term_id": "GO:0003777"
}